phosphatidylinositol phosphate phosphatase activity [GO:0052866] (molecular function) Definition: Catalysis of the reaction: phosphatidylinositol phosphate(n) + H2O = phosphatidylinositol phosphate(n-1) + phosphate. This reaction is the removal of a phosphate group from a phosphatidylinositol phosphate. Sources: GOC:ai Relationships: is a type of GO:0016791 Also known as: phosphoinositide phosphatase activity Subtypes: GO:0034593, phosphatidylinositol trisphosphate phosphatase activity [GO:0034594], phosphatidylinositol phosphate 5-phosphatase activity [GO:0034595], GO:0034596, phosphatidylinositol monophosphate phosphatase activity [GO:0052744]